regulation of trehalose metabolic process [GO:0090062] (biological process) Definition: Any process that modulates the frequency, rate or extent of trehalose metabolism, the chemical reactions and pathways involving trehalose, a disaccharide that consists of two molecules of glucose and is isomeric with sucrose. Relationships: is a type of regulation of carbohydrate metabolic process [GO:0006109]; regulates GO:0005991 Sources: GOC:dph, GOC:tb Subtypes: positive regulation of trehalose catabolic process [GO:1901319]